{
  "term_label": "Unknown molecular function",
  "gene": "UniProtKB:Q6S9Z5",
  "term_id": "UNKNOWN:0001",
  "gene_symbol": "ZNF474",
  "gene_name": "Zinc finger protein 474"
}